oxysterol 7-alpha-hydroxylase activity [GO:0008396] (molecular function) Relationships: is a type of steroid 7-alpha-hydroxylase activity [GO:0008387] Also known as: cytochrome P450 CYP7B1 Definition: Catalysis of the reaction: 7-oxocholesterol + H+ + NADPH = 7alpha-hydroxycholesterol + NADP+. Sources: RHEA:68740